leg disc anterior/posterior lineage restriction [GO:0035201] (biological process) Relationships: is a type of anterior/posterior lineage restriction, imaginal disc [GO:0048099]; is part of leg disc anterior/posterior pattern formation [GO:0035200] Definition: Formation and/or maintenance of a lineage boundary between anterior and posterior compartments of the leg disc that cells cannot cross, thus separating the populations of cells in each compartment. Sources: GOC:bf